{
  "gene_name": "Protein transport protein Sec23B",
  "term_id": "GO:0090110",
  "gene": "UniProtKB:Q15437",
  "term_label": "COPII-coated vesicle cargo loading",
  "gene_symbol": "SEC23B"
}